{
  "term_id": "GO:0005886",
  "gene_name": "Rap guanine nucleotide exchange factor 6",
  "gene": "UniProtKB:Q8TEU7",
  "gene_symbol": "RAPGEF6",
  "term_label": "plasma membrane"
}